{
  "term_label": "RNA polymerase II cis-regulatory region sequence-specific DNA binding",
  "gene_symbol": "ZNF883",
  "term_id": "GO:0000978",
  "gene": "UniProtKB:P0CG24",
  "gene_name": "Zinc finger protein 883"
}